{
  "gene_symbol": "FGF17",
  "term_id": "GO:0008284",
  "gene": "UniProtKB:O60258",
  "gene_name": "Fibroblast growth factor 17",
  "term_label": "positive regulation of cell population proliferation"
}